actin filament capping [GO:0051693] (biological process) Definition: The binding of a protein or protein complex to the end of an actin filament, thus preventing the addition, exchange or removal of further actin subunits. Sources: ISBN:071673706X Subtypes: barbed-end actin filament capping [GO:0051016], GO:0051694 Also known as: F-actin capping activity, actin capping activity Relationships: is a type of negative regulation of actin filament depolymerization [GO:0030835]; is a type of GO:0030837